{
  "term_id": "GO:0048179",
  "gene": "UniProtKB:P36896",
  "term_label": "activin receptor complex",
  "gene_symbol": "ACVR1B",
  "gene_name": "Activin receptor type-1B"
}